{
  "term_label": "dendrite",
  "gene": "UniProtKB:P35367",
  "gene_symbol": "HRH1",
  "gene_name": "Histamine H1 receptor",
  "term_id": "GO:0030425"
}